{
  "gene_name": "E3 ubiquitin-protein ligase CHFR",
  "term_label": "ubiquitin-dependent protein catabolic process",
  "gene_symbol": "CHFR",
  "gene": "UniProtKB:Q96EP1",
  "term_id": "GO:0006511"
}